{
  "term_id": "GO:0034361",
  "term_label": "very-low-density lipoprotein particle",
  "gene_name": "Apolipoprotein A-I",
  "gene_symbol": "APOA1",
  "gene": "UniProtKB:P02647"
}